{
  "term_label": "purine nucleotide biosynthetic process",
  "gene_name": "Ribose-phosphate pyrophosphokinase 2",
  "term_id": "GO:0006164",
  "gene": "UniProtKB:P11908",
  "gene_symbol": "PRPS2"
}